{
  "term_label": "Unknown cellular component",
  "gene": "UniProtKB:P28698",
  "gene_symbol": "MZF1",
  "gene_name": "Myeloid zinc finger 1",
  "term_id": "UNKNOWN:0003"
}